{
  "term_label": "extracellular space",
  "gene_symbol": "BMPER",
  "gene_name": "BMP-binding endothelial regulator protein",
  "gene": "UniProtKB:Q8N8U9",
  "term_id": "GO:0005615"
}